DNA-templated transcription elongation [GO:0006354] (BP) Definition: The extension of an RNA molecule after transcription initiation and promoter clearance at a DNA-dependent RNA polymerase promoter by the addition of ribonucleotides catalyzed by an RNA polymerase. Also known as: RNA elongation, DNA-dependent transcription, elongation, DNA-templated transcription, elongation, transcription elongation, DNA-dependent, transcriptional elongation, DNA-dependent, RNA elongation from bacterial-type RNA polymerase promoter, transcription elongation from bacterial-type RNA polymerase promoter Regulation: regulated by regulation of DNA-templated transcription elongation [GO:0032784]; negatively regulated by negative regulation of DNA-templated transcription, elongation [GO:0032785]; positively regulated by positive regulation of DNA-templated transcription, elongation [GO:0032786] Relationships: is a type of RNA biosynthetic process [GO:0032774]; BFO_0000050 DNA-templated transcription [GO:0006351] Subtypes: GO:0006362, transcription elongation by RNA polymerase II [GO:0006368], GO:0006385, transcription elongation by mitochondrial RNA polymerase [GO:0006392] References: PMID:15020047, PMID:18280161 Sources: GOC:mah, GOC:txnOH